{
  "gene_name": "Semaphorin-4C",
  "term_label": "semaphorin receptor binding",
  "term_id": "GO:0030215",
  "gene_symbol": "SEMA4C",
  "gene": "UniProtKB:Q9C0C4"
}